negative regulation of arugosin biosynthetic process [GO:1900627] (biological process) Definition: Any process that stops, prevents or reduces the frequency, rate or extent of arugosin biosynthetic process. Sources: GOC:TermGenie, GOC:di Also known as: down regulation of arugosin anabolism, down regulation of arugosin biosynthesis, down regulation of arugosin biosynthetic process, down regulation of arugosin formation, down regulation of arugosin synthesis, down-regulation of arugosin anabolism, down-regulation of arugosin biosynthesis, down-regulation of arugosin biosynthetic process, down-regulation of arugosin formation, down-regulation of arugosin synthesis, downregulation of arugosin anabolism, downregulation of arugosin biosynthesis, downregulation of arugosin biosynthetic process, downregulation of arugosin formation, downregulation of arugosin synthesis, inhibition of arugosin anabolism, inhibition of arugosin biosynthesis, inhibition of arugosin formation, inhibition of arugosin synthesis, negative regulation of arugosin anabolism, negative regulation of arugosin biosynthesis, negative regulation of arugosin formation, negative regulation of arugosin synthesis, inhibition of arugosin biosynthetic process Relationships: is a type of GO:1900377; is a type of regulation of arugosin biosynthetic process [GO:1900626]; negatively regulates arugosin biosynthetic process [GO:1900587]